{
  "term_id": "GO:0051321",
  "term_label": "meiotic cell cycle",
  "gene_name": "Protein FAM9C",
  "gene": "UniProtKB:Q8IZT9",
  "gene_symbol": "FAM9C"
}